{
  "term_id": "GO:0016020",
  "gene_symbol": "TGFBRAP1",
  "gene": "UniProtKB:Q8WUH2",
  "term_label": "membrane",
  "gene_name": "Transforming growth factor-beta receptor-associated protein 1"
}